establishment of glial blood-brain barrier [GO:0060857] (biological process) References: PMID:20080302 Sources: GOC:dph, GOC:sart Relationships: is a type of GO:0021782; is a type of establishment of blood-brain barrier [GO:0060856] Also known as: establishment of glial BBB, establishment of glial blood/brain barrier Definition: Establishment of the glial barrier between the blood and the brain. The glial cells in the brain are packed tightly together preventing the passage of most molecules from the blood into the brain. Only lipid soluble molecules or those that are actively transported can pass through the blood-brain barrier.